{
  "gene": "UniProtKB:Q9P2N6",
  "term_id": "GO:0045944",
  "gene_name": "KAT8 regulatory NSL complex subunit 3",
  "term_label": "positive regulation of transcription by RNA polymerase II",
  "gene_symbol": "KANSL3"
}